{
  "gene_symbol": "FLOT2",
  "gene": "UniProtKB:Q14254",
  "term_label": "protease binding",
  "term_id": "GO:0002020",
  "gene_name": "Flotillin-2"
}